regulation of activated T cell proliferation [GO:0046006] (biological process) Definition: Any process that modulates the frequency, rate or extent of activated T cell proliferation. Sources: GOC:go_curators Also known as: regulation of activated T lymphocyte proliferation, regulation of activated T-cell proliferation, regulation of activated T-lymphocyte proliferation Relationships: is a type of regulation of T cell proliferation [GO:0042129]; regulates activated T cell proliferation [GO:0050798] Subtypes: GO:0042104, GO:0046007